{
  "term_label": "Unknown biological process",
  "gene_name": "Cystatin-C",
  "gene_symbol": "CST3",
  "gene": "UniProtKB:P01034",
  "term_id": "UNKNOWN:0002"
}